{
  "gene_name": "ADP_ATP translocase 2",
  "term_label": "mitochondrial permeability transition pore complex",
  "term_id": "GO:0005757",
  "gene": "UniProtKB:P05141",
  "gene_symbol": "SLC25A5"
}